{
  "gene": "UniProtKB:Q6PIJ6",
  "gene_symbol": "FBXO38",
  "term_id": "GO:0005737",
  "gene_name": "F-box only protein 38",
  "term_label": "cytoplasm"
}